{
  "gene": "UniProtKB:Q8TEK3",
  "gene_name": "Histone-lysine N-methyltransferase, H3 lysine-79 specific",
  "gene_symbol": "DOT1L",
  "term_id": "GO:0031151",
  "term_label": "histone H3K79 methyltransferase activity"
}